{
  "term_label": "filopodium assembly",
  "gene_symbol": "SPAG6",
  "gene": "UniProtKB:O75602",
  "term_id": "GO:0046847",
  "gene_name": "Sperm-associated antigen 6"
}